{
  "gene_name": "Sulfotransferase 1A3",
  "term_id": "GO:0004062",
  "term_label": "aryl sulfotransferase activity",
  "gene_symbol": "SULT1A3",
  "gene": "UniProtKB:P0DMM9"
}